{
  "gene": "UniProtKB:Q96TC7",
  "gene_symbol": "RMDN3",
  "term_id": "GO:0097431",
  "gene_name": "Regulator of microtubule dynamics protein 3",
  "term_label": "mitotic spindle pole"
}